{
  "term_id": "GO:0048240",
  "gene_name": "Monoacylglycerol lipase ABHD2",
  "gene_symbol": "ABHD2",
  "gene": "UniProtKB:P08910",
  "term_label": "sperm capacitation"
}